{
  "gene_name": "Protocadherin-1",
  "gene": "UniProtKB:Q08174",
  "term_label": "cell adhesion",
  "gene_symbol": "PCDH1",
  "term_id": "GO:0007155"
}